{
  "gene": "UniProtKB:Q9H1X1",
  "gene_symbol": "RSPH9",
  "term_label": "cilium movement involved in cell motility",
  "term_id": "GO:0060294",
  "gene_name": "Radial spoke head protein 9 homolog"
}